{
  "gene_symbol": "BAZ1A",
  "gene": "UniProtKB:Q9NRL2",
  "term_label": "nuclear chromosome",
  "term_id": "GO:0000228",
  "gene_name": "Bromodomain adjacent to zinc finger domain protein 1A"
}